{
  "gene_name": "2-oxoglutarate receptor 1",
  "gene_symbol": "OXGR1",
  "term_label": "plasma membrane",
  "gene": "UniProtKB:Q96P68",
  "term_id": "GO:0005886"
}